{
  "gene": "UniProtKB:O60759",
  "gene_symbol": "CYTIP",
  "term_label": "cell cortex",
  "term_id": "GO:0005938",
  "gene_name": "Cytohesin-interacting protein"
}